{
  "term_id": "GO:0006357",
  "term_label": "regulation of transcription by RNA polymerase II",
  "gene": "UniProtKB:P42224",
  "gene_name": "Signal transducer and activator of transcription 1-alpha_beta",
  "gene_symbol": "STAT1"
}